{
  "term_label": "U2 snRNP",
  "gene_symbol": "SNRPA1",
  "term_id": "GO:0005686",
  "gene_name": "U2 small nuclear ribonucleoprotein A'",
  "gene": "UniProtKB:P09661"
}